{
  "gene_name": "Myoglobin",
  "term_id": "GO:0019430",
  "term_label": "removal of superoxide radicals",
  "gene": "UniProtKB:P02144",
  "gene_symbol": "MB"
}